peripheral nervous system axon regeneration [GO:0014012] (biological process) Sources: GOC:ef Relationships: is a type of axon regeneration [GO:0031103] Also known as: axon regeneration in peripheral nervous system Definition: The regrowth of axons outside the central nervous system (outside the brain and spinal cord) following an axonal injury.